meiotic S phase [GO:0051332] (biological process) Also known as: S phase of meiotic cell cycle, S-phase of meiotic cell cycle, premeiotic S-phase Note: Note that this term should not be used for direct annotation. If you are trying to make an annotation to x phase, it is likely that the correct annotation is 'regulation of x/y phase transition' or to a process which occurs during the reported phase (i.e mitotic DNA replication for mitotic S-phase). To capture the phase when a specific location or process is observed, the phase term can be used in an annotation extension (PMID:24885854) applied to a cellular component term (with the relation exists_during) or a biological process term (with the relation happens_during). Relationships: is_a S phase [GO:0051320]; is part of meiotic interphase [GO:0051328] Definition: The cell cycle phase, following G1, during which DNA synthesis takes place as part of a meiotic cell cycle. Sources: GOC:mtg_cell_cycle